hexose:proton symporter activity [GO:0009679] (MF) Also known as: hexose:hydrogen symporter activity Definition: Enables the transfer of a solute or solutes from one side of a membrane to the other according to the reaction: hexose(out) + H+(out) = hexose(in) + H+(in). Relationships: is a type of GO:0005351; is a type of hexose transmembrane transporter activity [GO:0015149] Subtypes: D-glucose:proton symporter activity [GO:0005356], galactose:proton symporter activity [GO:0015517], GO:0015535, rhamnose:proton symporter activity [GO:0015561], mannose:proton symporter activity [GO:0055053], fructose:proton symporter activity [GO:0055054] Sources: TC:2.A.1.-.-